{
  "term_label": "plasma membrane",
  "gene": "UniProtKB:Q96CP6",
  "gene_symbol": "GRAMD1A",
  "term_id": "GO:0005886",
  "gene_name": "Protein Aster-A"
}